{
  "term_label": "nucleus",
  "term_id": "GO:0005634",
  "gene_name": "Protein FAM50A",
  "gene": "UniProtKB:Q14320",
  "gene_symbol": "FAM50A"
}